histone H4K20me methyltransferase activity [GO:0140941] (molecular function) Relationships: is a type of histone H4K20 methyltransferase activity [GO:0042799] Definition: Catalysis of the reaction: N(6)-methyl-L-lysyl(20)-[histone H4] + S-adenosyl-L-methionine = H+ + N(6),N(6)-dimethyl-L-lysyl(20)-[histone H4] + S-adenosyl-L-homocysteine. This reaction is the addition of a methyl group to the monomethylated lysine residue at position 20 of histone H4, producing H4K20me2. Also known as: histone H4-K20 dimethylation, histone H4K20 dimethylation, histone H4 methyl lysine(20) N-methyltransferase activity (H4-K20 specific), histone H4K20me methylase activity Sources: RHEA:60348 Note: Note that the residue position corresponds to the canonical human H4 histone (UniProtKB:P02309); this residue is conserved across all eukaryotes. Note that the initiation methionine is cleaved, so the first residue is S1.